radial spoke head [GO:0001535] (cellular component) Also known as: radial spokehead Relationships: is a type of protein-containing complex [GO:0032991]; is part of GO:0001534 Definition: Protein complex forming portion of the radial spoke that is orthogonal to the elongated stalk and which projects towards the central pair of microtubules within the ciliary or flagellum axoneme. References: PMID:22754630, PMID:34871179 Sources: GOC:cilia, GOC:hjd, GOC:krc Subtypes: GO:0120336, radial spoke head 2 [GO:0120337], GO:0120338